response to ceramide [GO:0106096] (biological process) References: PMID:18006463 Definition: Any process that results in a change in state or activity of a cell or an organism (in terms of movement, secretion, enzyme production, gene expression, etc.) as a result of a ceramide stimulus. Relationships: is a type of response to lipid [GO:0033993]